UDP-glycosyltransferase activity [GO:0008194] (molecular function) Relationships: is a type of glycosyltransferase activity [GO:0016757] References: PMID:11846783 Subtypes: acetylglucosaminyltransferase activity [GO:0008375], GO:0008376, GO:0008915, glucuronosyltransferase activity [GO:0015020], UDP-galactosyltransferase activity [GO:0035250], GO:0035251, UDP-xylosyltransferase activity [GO:0035252], GO:0046510, flavonol-3-O-glucoside L-rhamnosyltransferase activity [GO:0047230], lipopolysaccharide N-acetylmannosaminouronosyltransferase activity [GO:0047241], N-acetylglucosaminyldiphosphoundecaprenol N-acetyl-beta-D-mannosaminyltransferase activity [GO:0047244], diglucosyl diacylglycerol synthase activity [GO:0047257], polygalacturonate 4-alpha-galacturonosyltransferase activity [GO:0047262], 1,4-beta-D-xylan synthase activity [GO:0047517], alpha-1,3-glucan synthase activity [GO:0047657], flavone apiosyltransferase activity [GO:0047892], linamarin synthase activity [GO:0050057], indolylacetylinositol arabinosyltransferase activity [GO:0050409], hyaluronan synthase activity [GO:0050501], flavonol 3-O-arabinosyltransferase activity [GO:0080059], sphingolipid alpha-glucuronosyltransferase activity [GO:1990482] Definition: Catalysis of the transfer of a glycosyl group from a UDP-sugar to a small hydrophobic molecule.